{
  "gene": "UniProtKB:Q15907",
  "term_id": "GO:0045054",
  "term_label": "constitutive secretory pathway",
  "gene_symbol": "RAB11B",
  "gene_name": "Ras-related protein Rab-11B"
}